{
  "gene_name": "Receptor-type tyrosine-protein phosphatase F",
  "gene": "UniProtKB:P10586",
  "term_label": "Unknown cellular component",
  "gene_symbol": "PTPRF",
  "term_id": "UNKNOWN:0003"
}